{
  "term_label": "chromatin remodeling",
  "term_id": "GO:0006338",
  "gene_symbol": "RBBP7",
  "gene_name": "Histone-binding protein RBBP7",
  "gene": "UniProtKB:Q16576"
}